{
  "term_id": "GO:0098978",
  "gene": "UniProtKB:P98172",
  "gene_symbol": "EFNB1",
  "term_label": "glutamatergic synapse",
  "gene_name": "Ephrin-B1"
}